{
  "term_label": "regulation of cell cycle",
  "gene_symbol": "CDK7",
  "term_id": "GO:0051726",
  "gene_name": "Cyclin-dependent kinase 7",
  "gene": "UniProtKB:P50613"
}